S-adenosyl-L-methionine:S-adenosyl-L-homocysteine antiporter activity [GO:0180003] (molecular function) References: PMID:14674884, PMID:34375635 Definition: Catalysis of the reaction: S-adenosyl-L-homocysteine(out) + S-adenosyl-L-methionine(in) = S-adenosyl-L-homocysteine(in) + S-adenosyl-L-methionine(out). Relationships: is a type of GO:0000095; is a type of GO:0015179; is a type of purine nucleoside transmembrane transporter activity [GO:0015211]; is a type of GO:0015297; is a type of GO:0072349